{
  "gene": "UniProtKB:P51636",
  "gene_name": "Caveolin-2",
  "gene_symbol": "CAV2",
  "term_label": "caveola",
  "term_id": "GO:0005901"
}